{
  "term_label": "Unknown molecular function",
  "gene": "UniProtKB:Q5T890",
  "gene_name": "DNA excision repair protein ERCC-6-like 2",
  "term_id": "UNKNOWN:0001",
  "gene_symbol": "ERCC6L2"
}